arsenite secondary active transmembrane transporter activity [GO:0008490] (molecular function) Sources: GOC:jl Definition: Enables the transfer of arsenite from one side of a membrane to the other, up its concentration gradient. The transporter binds the solute and undergoes a series of conformational changes. Transport works equally well in either direction and is driven by a chemiosmotic source of energy. Secondary active transporters include symporters and antiporters. Relationships: is a type of arsenite transmembrane transporter activity [GO:0015105]; is a type of secondary active transmembrane transporter activity [GO:0015291] Also known as: arsenite porter activity